striated muscle paramyosin thick filament assembly [GO:0061203] (biological process) Definition: The aggregation, arrangement and bonding together of proteins to form the paramyosin-based thick filaments of myofibrils in striated muscle. Sources: GOC:dph, GOC:kmv Relationships: is a type of paramyosin filament assembly or disassembly [GO:0061204]; is part of myofibril assembly [GO:0030239]